{
  "gene_name": "Low-density lipoprotein receptor-related protein 8",
  "term_label": "plasma membrane",
  "gene_symbol": "LRP8",
  "gene": "UniProtKB:Q14114",
  "term_id": "GO:0005886"
}